tiggrin receptor activity [GO:0005056] (molecular function) Definition: Combining with the extracellular matrix ligand tiggrin, and transmitting the signal from one side of the membrane to the other to initiate a change in cell activity. Relationships: is_a transmembrane signaling receptor activity [GO:0004888] References: PMID:9521906 Sources: GOC:mah, GOC:signaling